{
  "term_label": "Unknown molecular function",
  "gene_symbol": "TEKT5",
  "gene": "UniProtKB:Q96M29",
  "gene_name": "Tektin-5",
  "term_id": "UNKNOWN:0001"
}